nucleotide salvage [GO:0043173] (biological process) Definition: Any process which produces a nucleotide, a compound consisting of a nucleoside that is esterified with (ortho)phosphate or an oligophosphate at any hydroxyl group on the glycose moiety, from derivatives of it without de novo synthesis. Sources: GOC:jl Relationships: is a type of nucleotide biosynthetic process [GO:0009165]; is a type of metabolic compound salvage [GO:0043094] Subtypes: pyridine nucleotide salvage [GO:0019365], GO:0032261, pyrimidine nucleotide salvage [GO:0032262]